{
  "gene_symbol": "TRIM42",
  "term_id": "UNKNOWN:0003",
  "term_label": "Unknown cellular component",
  "gene_name": "Tripartite motif-containing protein 42",
  "gene": "UniProtKB:Q8IWZ5"
}